glucosinolate:proton symporter activity [GO:0090448] (molecular function) References: PMID:22864417 Definition: Enables the transfer of a solute or solutes from one side of a membrane to the other according to the reaction: glucosinolate(out) + H+(out) = glucosinolate(in) + H+(in). Relationships: is a type of solute:proton symporter activity [GO:0015295]; is a type of glucosinolate transmembrane transporter activity [GO:0141165] Also known as: glucosinolate:hydrogen symporter activity